regulation of timing of plant organ formation [GO:0090709] (biological process) Definition: Any process that modulates the rate, frequency or extent of plant organ formation at a consistent predetermined time point during development. Relationships: is a type of regulation of development, heterochronic [GO:0040034]; is a type of GO:1905428 Sources: GOC:tb